{
  "gene_symbol": "MTNR1A",
  "gene": "UniProtKB:P48039",
  "gene_name": "Melatonin receptor type 1A",
  "term_label": "plasma membrane",
  "term_id": "GO:0005886"
}